{
  "gene": "UniProtKB:P49721",
  "gene_name": "Proteasome subunit beta type-2",
  "term_label": "proteasome core complex, beta-subunit complex",
  "gene_symbol": "PSMB2",
  "term_id": "GO:0019774"
}